negative regulation of apical ectodermal ridge formation [GO:1905141] (biological process) Definition: Any process that stops, prevents or reduces the frequency, rate or extent of apical ectodermal ridge formation. Also known as: down regulation of apical ectodermal ridge formation, down regulation of apical epidermal ridge formation, down-regulation of apical ectodermal ridge formation, down-regulation of apical epidermal ridge formation, downregulation of apical ectodermal ridge formation, downregulation of apical epidermal ridge formation, negative regulation of apical epidermal ridge formation, inhibition of apical ectodermal ridge formation, inhibition of apical epidermal ridge formation, down regulation of AER formation, down regulation of crista ectodermalis apicalis formation, down-regulation of AER formation, down-regulation of crista ectodermalis apicalis formation, downregulation of AER formation, downregulation of crista ectodermalis apicalis formation, inhibition of AER formation, inhibition of crista ectodermalis apicalis formation, negative regulation of AER formation, negative regulation of crista ectodermalis apicalis formation References: PMID:18359901 Sources: GOC:TermGenie, GO_REF:0000058 Relationships: is a type of negative regulation of developmental process [GO:0051093]; is a type of GO:0051241; is a type of regulation of apical ectodermal ridge formation [GO:1905140]; negatively regulates apical ectodermal ridge formation [GO:1905139]